(-)-secoisolariciresinol biosynthetic process [GO:1902138] (biological process) Relationships: is a type of lignan biosynthetic process [GO:0009807]; is a type of diol biosynthetic process [GO:0034312]; is a type of phenol-containing compound biosynthetic process [GO:0046189] Also known as: (-)-secoisolariciresinol anabolism, (-)-secoisolariciresinol biosynthesis, (-)-secoisolariciresinol formation, (-)-secoisolariciresinol synthesis Definition: The chemical reactions and pathways resulting in the formation of (-)-secoisolariciresinol. References: PMID:8910615, PMID:9872995 Sources: GOC:TermGenie